{
  "gene_symbol": "ARHGAP30",
  "gene_name": "Rho GTPase-activating protein 30",
  "term_label": "small GTPase-mediated signal transduction",
  "gene": "UniProtKB:Q7Z6I6",
  "term_id": "GO:0007264"
}